positive regulation of intraciliary anterograde transport [GO:1905798] (biological process) Also known as: positive regulation of intraflagellar anterograde transport, up regulation of intraciliary anterograde transport, up regulation of intraflagellar anterograde transport, up-regulation of intraciliary anterograde transport, up-regulation of intraflagellar anterograde transport, upregulation of intraciliary anterograde transport, upregulation of intraflagellar anterograde transport, activation of intraciliary anterograde transport, activation of intraflagellar anterograde transport Relationships: is a type of GO:0010638; is a type of GO:0032388; is a type of regulation of intraciliary anterograde transport [GO:1905796]; positively regulates intraciliary anterograde transport [GO:0035720] Definition: Any process that activates or increases the frequency, rate or extent of intraciliary anterograde transport. References: PMID:27930654 Sources: GOC:TermGenie, GO_REF:0000058